{
  "gene_name": "T cell receptor beta variable 6-9",
  "term_id": "GO:0005886",
  "term_label": "plasma membrane",
  "gene_symbol": "TRBV6-9",
  "gene": "UniProtKB:A0A0J9YX75"
}